telomere maintenance [GO:0000723] (biological process) Definition: Any process that contributes to the maintenance of proper telomeric length and structure by affecting and monitoring the activity of telomeric proteins, the length of telomeric DNA and the replication and repair of the DNA. These processes includes those that shorten, lengthen, replicate and repair the telomeric DNA sequences. References: PMID:11092831 Sources: GOC:BHF, GOC:BHF_telomere, GOC:elh, GOC:rl Also known as: regulation of telomere length Relationships: is a type of DNA metabolic process [GO:0006259]; is a type of telomere organization [GO:0032200] Subtypes: telomere maintenance via recombination [GO:0000722], GO:0010833, telomere capping [GO:0016233], telomeric loop formation [GO:0031627], GO:0032201, telomere maintenance in response to DNA damage [GO:0043247], telomeric loop disassembly [GO:0090657], telomere maintenance via telomere trimming [GO:0090737] Regulation: regulated by regulation of telomere maintenance [GO:0032204]; negatively regulated by GO:0032205; RO_0002213 by GO:0032206